desacetoxyvindoline 4-hydroxylase activity [GO:0050590] (molecular function) Sources: EC:1.14.11.20, MetaCyc:1.14.11.20-RXN Also known as: D17H activity, deacetoxyvindoline,2-oxoglutarate:oxygen oxidoreductase (4beta-hydroxylating), desacetoxyvindoline,2-oxoglutarate:oxygen oxidoreductase (4-beta-hydroxylating) activity, desacetoxyvindoline,2-oxoglutarate:oxygen oxidoreductase (4beta-hydroxylating), desacetoxyvindoline-4-hydroxylase activity, desacetyoxyvindoline-17-hydroxylase activity Definition: Catalysis of the reaction: desacetoxyvindoline + 2-oxoglutarate + O2 = desacetylvindoline + succinate + CO2. Relationships: is a type of 2-oxoglutarate-dependent dioxygenase activity [GO:0016706]